NAD+ poly-ADP-ribosyltransferase activity [GO:0003950] (molecular function) Relationships: is a type of pentosyltransferase activity [GO:0016763] Also known as: NAD+ ADP-ribosyltransferase activity, NAD ADP-ribosyltransferase activity, NAD+-protein poly-ADP-ribosyltransferase activity, ADP-ribosyltransferase (polymerizing) activity, NAD+:poly(adenine-diphosphate-D-ribosyl)-acceptor ADP-D-ribosyl-transferase activity, poly(ADP-ribose) synthase activity, poly(ADP-ribose) synthetase activity, poly(ADP-ribose)polymerase activity, poly(adenosine diphosphate ribose) polymerase activity Definition: Catalysis of the reaction: NAD+ + (ADP-D-ribosyl)(n)-acceptor = nicotinamide + (ADP-D-ribosyl)(n+1)-acceptor. Sources: EC:2.4.2.30